positive regulation of succinate dehydrogenase activity [GO:1904231] (biological process) Relationships: is a type of positive regulation of oxidoreductase activity [GO:0051353]; positively regulates succinate dehydrogenase activity [GO:0000104] Definition: Any process that activates or increases the frequency, rate or extent of succinate dehydrogenase activity. References: PMID:18160053 Sources: GOC:BHF, GOC:TermGenie, GOC:rl, GO_REF:0000059 Also known as: positive regulation of fumarate dehydrogenase activity, positive regulation of fumarate reductase activity, positive regulation of fumaric hydrogenase activity, positive regulation of succinate oxidoreductase activity, positive regulation of succinate:(acceptor) oxidoreductase activity, positive regulation of succinate:acceptor oxidoreductase activity, positive regulation of succinic acid dehydrogenase activity, positive regulation of succinodehydrogenase activity, positive regulation of succinyl dehydrogenase activity, up regulation of fumarate dehydrogenase activity, up regulation of fumarate reductase activity, up regulation of fumaric hydrogenase activity, up regulation of succinate dehydrogenase activity, up regulation of succinate oxidoreductase activity, up regulation of succinate:(acceptor) oxidoreductase activity, up regulation of succinate:acceptor oxidoreductase activity, up regulation of succinic acid dehydrogenase activity, up regulation of succinodehydrogenase activity, up regulation of succinyl dehydrogenase activity, up-regulation of fumarate dehydrogenase activity, up-regulation of fumarate reductase activity, up-regulation of fumaric hydrogenase activity, up-regulation of succinate dehydrogenase activity, up-regulation of succinate oxidoreductase activity, up-regulation of succinate:(acceptor) oxidoreductase activity, up-regulation of succinate:acceptor oxidoreductase activity, up-regulation of succinic acid dehydrogenase activity, up-regulation of succinodehydrogenase activity, up-regulation of succinyl dehydrogenase activity, upregulation of fumarate dehydrogenase activity, upregulation of fumarate reductase activity, upregulation of fumaric hydrogenase activity, upregulation of succinate dehydrogenase activity, upregulation of succinate oxidoreductase activity, upregulation of succinate:(acceptor) oxidoreductase activity, upregulation of succinate:acceptor oxidoreductase activity, upregulation of succinic acid dehydrogenase activity, upregulation of succinodehydrogenase activity, upregulation of succinyl dehydrogenase activity, activation of fumarate dehydrogenase activity, activation of fumarate reductase activity, activation of fumaric hydrogenase activity, activation of succinate dehydrogenase activity, activation of succinate oxidoreductase activity, activation of succinate:(acceptor) oxidoreductase activity, activation of succinate:acceptor oxidoreductase activity, activation of succinic acid dehydrogenase activity, activation of succinodehydrogenase activity, activation of succinyl dehydrogenase activity